{
  "gene_symbol": "ATF1",
  "term_id": "GO:0141156",
  "gene_name": "Cyclic AMP-dependent transcription factor ATF-1",
  "gene": "UniProtKB:P18846",
  "term_label": "cAMP/PKA signal transduction"
}